{
  "term_label": "Unknown cellular component",
  "term_id": "UNKNOWN:0003",
  "gene": "UniProtKB:Q8WZ84",
  "gene_name": "Olfactory receptor 8D1",
  "gene_symbol": "OR8D1"
}